{
  "term_label": "cytosol",
  "gene_symbol": "MAT1A",
  "term_id": "GO:0005829",
  "gene": "UniProtKB:Q00266",
  "gene_name": "S-adenosylmethionine synthase isoform type-1"
}